negative regulation of mammary gland epithelial cell proliferation [GO:0033600] (biological process) Also known as: down regulation of mammary gland epithelial cell proliferation, down-regulation of mammary gland epithelial cell proliferation, downregulation of mammary gland epithelial cell proliferation, inhibition of mammary gland epithelial cell proliferation Definition: Any process that stops, prevents or reduces the rate or extent of mammary gland epithelial cell proliferation. Sources: GOC:mah Relationships: is_a regulation of mammary gland epithelial cell proliferation [GO:0033599]; is a type of GO:0050680; is a type of negative regulation of multicellular organismal process [GO:0051241]; negatively regulates mammary gland epithelial cell proliferation [GO:0033598]